{
  "gene_name": "Putative transcription factor Ovo-like 1",
  "gene": "UniProtKB:O14753",
  "gene_symbol": "OVOL1",
  "term_id": "GO:0005634",
  "term_label": "nucleus"
}